{
  "gene_symbol": "PRPH2",
  "gene_name": "Peripherin-2",
  "term_id": "GO:0005886",
  "gene": "UniProtKB:P23942",
  "term_label": "plasma membrane"
}